membrane depolarization during atrial cardiac muscle cell action potential [GO:0098912] (biological process) Definition: The process in which atrial cardiac muscle cell membrane potential changes in the depolarizing direction from the negative resting potential towards the positive membrane potential that will be the peak of the action potential. Sources: GOC:dph, GOC:mtg_cardiac_conduct_nov11, GOC:tb Also known as: atrial cardiac muscle cell depolarization, atrial depolarization, electrocardiogram PR interval Relationships: is a type of membrane depolarization during cardiac muscle cell action potential [GO:0086012]; BFO_0000050 GO:0086014